{
  "gene_symbol": "COG8",
  "term_id": "GO:0006891",
  "gene_name": "Conserved oligomeric Golgi complex subunit 8",
  "term_label": "intra-Golgi vesicle-mediated transport",
  "gene": "UniProtKB:Q96MW5"
}